{
  "term_id": "GO:0004930",
  "gene": "UniProtKB:P32745",
  "term_label": "G protein-coupled receptor activity",
  "gene_name": "Somatostatin receptor type 3",
  "gene_symbol": "SSTR3"
}